{
  "term_label": "tRNA processing",
  "gene_symbol": "POP7",
  "gene_name": "Ribonuclease P protein subunit p20",
  "term_id": "GO:0008033",
  "gene": "UniProtKB:O75817"
}